{
  "term_label": "Unknown cellular component",
  "gene": "UniProtKB:Q8NGI7",
  "term_id": "UNKNOWN:0003",
  "gene_name": "Olfactory receptor 10V1",
  "gene_symbol": "OR10V1"
}